n-octane oxidation [GO:0019498] (biological process) Relationships: is a type of xenobiotic catabolic process [GO:0042178] Sources: MetaCyc:P221-PWY Definition: The chemical reactions and pathways resulting in the conversion of n-octane to octanoyl-CoA.